{
  "gene": "UniProtKB:A0A0G2JRQ6",
  "term_id": "GO:0019814",
  "gene_name": "Ig-like domain-containing protein (Fragment)",
  "gene_symbol": "A0A0G2JRQ6",
  "term_label": "immunoglobulin complex"
}